{
  "gene_symbol": "PMVK",
  "term_id": "UNKNOWN:0003",
  "gene_name": "Phosphomevalonate kinase",
  "term_label": "Unknown cellular component",
  "gene": "UniProtKB:Q15126"
}